{
  "term_id": "GO:0005096",
  "gene_name": "Rho GTPase-activating protein 32",
  "gene": "UniProtKB:A7KAX9",
  "gene_symbol": "ARHGAP32",
  "term_label": "GTPase activator activity"
}